asexual sporulation [GO:0030436] (biological process) Also known as: asexual reproductive sporulation, asexual spore formation, mitotic spore formation, mitotic sporulation Subtypes: oidium formation [GO:0034297], asexual sporulation resulting in formation of a cellular spore [GO:0043936], conidium formation [GO:0048315], asexual sporulation resulting in formation of a multicellular or syncytial spore [GO:0075284], oomycete sporangium development [GO:0075321] Definition: The formation of spores derived from the products of an asexual cell division. Examples of this process are found in bacteria and fungi. References: PMID:9529886 Sources: GOC:mah Regulation: regulated by regulation of asexual sporulation [GO:0034305] Relationships: is a type of developmental process involved in reproduction [GO:0003006]; is a type of asexual reproduction [GO:0019954]; is a type of sporulation [GO:0043934]